response to red or far red light [GO:0009639] (biological process) Relationships: is a type of response to light stimulus [GO:0009416] Regulation: regulated by regulation of response to red or far red light [GO:2000030] Subtypes: photomorphogenesis [GO:0009640], shade avoidance [GO:0009641], response to red light [GO:0010114], GO:0010218, GO:0071489 Sources: GOC:ai, GOC:mtg_far_red Definition: Any process that results in a change in state or activity of a cell or an organism (in terms of movement, secretion, enzyme production, gene expression, etc.) as a result of a red or far red light stimulus. Red light is electromagnetic radiation of wavelength of 580-700nm. Far red light is electromagnetic radiation of wavelength 700-800nm. An example of this response is seen at the beginning of many plant species developmental stages. These include germination, and the point when cotyledon expansion is triggered. In certain species these processes take place in response to absorption of red light by the pigment molecule phytochrome, but the signal can be reversed by exposure to far red light. During the initial phase the phytochrome molecule is only present in the red light absorbing form, but on absorption of red light it changes to a far red light absorbing form, triggering progress through development. An immediate short period of exposure to far red light entirely returns the pigment to its initial state and prevents triggering of the developmental process. A thirty minute break between red and subsequent far red light exposure renders the red light effect irreversible, and development then occurs regardless of whether far red light exposure subsequently occurs.